regulation of peptidyl-tyrosine phosphorylation [GO:0050730] (biological process) Subtypes: regulation of tyrosine phosphorylation of STAT protein [GO:0042509], GO:0050731, negative regulation of peptidyl-tyrosine phosphorylation [GO:0050732], GO:0061097, GO:1900084 Sources: GOC:ai Relationships: is a type of regulation of protein phosphorylation [GO:0001932]; regulates peptidyl-tyrosine phosphorylation [GO:0018108] Definition: Any process that modulates the frequency, rate or extent of the phosphorylation of peptidyl-tyrosine.